{
  "term_label": "histone H3K9me2/3 reader activity",
  "gene_symbol": "CDY2A",
  "term_id": "GO:0062072",
  "gene": "UniProtKB:Q9Y6F7",
  "gene_name": "Testis-specific chromodomain protein Y 2"
}